{
  "gene": "UniProtKB:Q8NBJ7",
  "term_label": "Unknown biological process",
  "gene_name": "Inactive C-alpha-formylglycine-generating enzyme 2",
  "term_id": "UNKNOWN:0002",
  "gene_symbol": "SUMF2"
}